negative regulation of mRNA 3'-end processing [GO:0031441] (biological process) Definition: Any process that stops, prevents, or reduces the frequency, rate or extent of mRNA 3'-end processing. Sources: GOC:mah Relationships: is_a regulation of mRNA 3'-end processing [GO:0031440]; is a type of GO:0050686; negatively regulates GO:0031124 Also known as: down regulation of mRNA 3'-end processing, down-regulation of mRNA 3'-end processing, downregulation of mRNA 3'-end processing, inhibition of mRNA 3'-end processing